{
  "term_label": "Unknown molecular function",
  "gene_symbol": "MPZL3",
  "gene": "UniProtKB:Q6UWV2",
  "gene_name": "Myelin protein zero-like protein 3",
  "term_id": "UNKNOWN:0001"
}